{
  "gene": "UniProtKB:Q9H9E1",
  "term_id": "UNKNOWN:0001",
  "gene_symbol": "ANKRA2",
  "term_label": "Unknown molecular function",
  "gene_name": "Ankyrin repeat family A protein 2"
}